{
  "gene_symbol": "ZDHHC13",
  "gene": "UniProtKB:Q8IUH4",
  "term_label": "Unknown cellular component",
  "gene_name": "Palmitoyltransferase ZDHHC13",
  "term_id": "UNKNOWN:0003"
}